positive regulation of T-helper 17 cell differentiation [GO:2000321] (biological process) Also known as: positive regulation of T-helper 17 cell development Sources: GOC:BHF, GOC:mah Definition: Any process that activates or increases the frequency, rate or extent of T-helper 17 cell differentiation. Subtypes: positive regulation of T-helper 17 cell lineage commitment [GO:2000330] Relationships: is_a positive regulation of T-helper cell differentiation [GO:0045624]; is a type of positive regulation of T-helper 17 type immune response [GO:2000318]; is a type of GO:2000319; positively regulates T-helper 17 cell differentiation [GO:0072539]